{
  "gene_name": "Kelch-like protein 12",
  "term_label": "cytoplasm",
  "gene": "UniProtKB:Q53G59",
  "gene_symbol": "KLHL12",
  "term_id": "GO:0005737"
}